{
  "gene_name": "Thymic stromal cotransporter homolog",
  "gene_symbol": "SLC46A2",
  "term_id": "GO:0055085",
  "gene": "UniProtKB:Q9BY10",
  "term_label": "transmembrane transport"
}